{
  "gene_name": "Thioredoxin-like protein 4B",
  "gene": "UniProtKB:Q9NX01",
  "term_id": "GO:0046540",
  "gene_symbol": "TXNL4B",
  "term_label": "U4/U6 x U5 tri-snRNP complex"
}